establishment of planar polarity of embryonic epithelium [GO:0042249] (biological process) Definition: Coordinated organization of groups of cells in the plane of an embryonic epithelium, such that they all orient to similar coordinates. Sources: GOC:ascb_2009, GOC:dph, GOC:jl, GOC:tb Relationships: is a type of GO:0001736 Subtypes: establishment of planar polarity involved in neural tube closure [GO:0090177]